{
  "gene": "UniProtKB:Q7Z402",
  "term_id": "UNKNOWN:0002",
  "gene_name": "Transmembrane channel-like protein 7",
  "gene_symbol": "TMC7",
  "term_label": "Unknown biological process"
}